{
  "gene_symbol": "VTI1B",
  "gene_name": "Vesicle transport through interaction with t-SNAREs homolog 1B",
  "term_id": "GO:1903076",
  "term_label": "regulation of protein localization to plasma membrane",
  "gene": "UniProtKB:Q9UEU0"
}